PCNA-p21 complex [GO:0070557] (cellular component) References: PMID:7911228, PMID:7915843 Sources: GOC:mah Definition: A protein complex that contains the cyclin-dependent protein kinase inhibitor p21WAF1/CIP1 bound to PCNA; formation of the complex inhibits DNA replication. Relationships: is a type of GO:0140513